{
  "gene_symbol": "CTPS2",
  "gene_name": "CTP synthase 2",
  "term_id": "GO:0006241",
  "gene": "UniProtKB:Q9NRF8",
  "term_label": "CTP biosynthetic process"
}